{
  "term_label": "Unknown cellular component",
  "gene_name": "Leucine-rich repeat-containing G-protein coupled receptor 6",
  "gene": "UniProtKB:Q9HBX8",
  "gene_symbol": "LGR6",
  "term_id": "UNKNOWN:0003"
}